ammonium channel activity [GO:0008519] (molecular function) Also known as: ammonia transmembrane transporter activity, ammonium transmembrane transporter activity Relationships: is a type of channel activity [GO:0015267]; is part of ammonium transmembrane transport [GO:0072488] References: PMID:17710640 Definition: Enables the energy-independent facilitated diffusion of ammonium through a transmembrane aqueous pore or channel.